{
  "term_id": "GO:1905606",
  "gene_symbol": "LRRC4B",
  "gene": "UniProtKB:Q9NT99",
  "gene_name": "Leucine-rich repeat-containing protein 4B",
  "term_label": "regulation of presynapse assembly"
}